{
  "gene": "UniProtKB:P41220",
  "term_id": "GO:0005096",
  "term_label": "GTPase activator activity",
  "gene_name": "Regulator of G-protein signaling 2",
  "gene_symbol": "RGS2"
}